glycine dehydrogenase activity [GO:0047960] (molecular function) Definition: Catalysis of the reaction: glycine + H2O + NAD+ = glyoxylate + NH3 + NADH. Sources: EC:1.4.1.10, MetaCyc:GLYCINE-DEHYDROGENASE-RXN Also known as: glycine:NAD+ oxidoreductase (deaminating) Relationships: is a type of oxidoreductase activity, acting on the CH-NH2 group of donors, NAD or NADP as acceptor [GO:0016639]